{
  "term_id": "GO:0043161",
  "gene": "UniProtKB:Q96B02",
  "term_label": "proteasome-mediated ubiquitin-dependent protein catabolic process",
  "gene_name": "Ubiquitin-conjugating enzyme E2 W",
  "gene_symbol": "UBE2W"
}